{
  "term_id": "UNKNOWN:0003",
  "gene_symbol": "TCP10L",
  "gene_name": "T-complex protein 10A homolog 1",
  "term_label": "Unknown cellular component",
  "gene": "UniProtKB:Q8TDR4"
}